{
  "term_id": "GO:0003729",
  "term_label": "mRNA binding",
  "gene_name": "Heterogeneous nuclear ribonucleoprotein A0",
  "gene": "UniProtKB:Q13151",
  "gene_symbol": "HNRNPA0"
}